{
  "gene": "UniProtKB:Q6ZMS4",
  "gene_name": "Zinc finger protein 852",
  "term_id": "GO:0006357",
  "term_label": "regulation of transcription by RNA polymerase II",
  "gene_symbol": "ZNF852"
}